{
  "gene_symbol": "LIPM",
  "gene_name": "Lipase member M",
  "term_label": "lipid metabolic process",
  "gene": "UniProtKB:Q5VYY2",
  "term_id": "GO:0006629"
}